{
  "term_label": "negative regulation of small GTPase mediated signal transduction",
  "gene": "UniProtKB:Q9Y3L3",
  "term_id": "GO:0051058",
  "gene_symbol": "SH3BP1",
  "gene_name": "SH3 domain-binding protein 1"
}